sulfotransferase activity [GO:0008146] (molecular function) Relationships: is a type of transferase activity, transferring sulphur-containing groups [GO:0016782] Also known as: sulphotransferase activity Sources: EC:2.8.2.- Subtypes: N-acetylglucosamine 6-O-sulfotransferase activity [GO:0001517], alcohol sulfotransferase activity [GO:0004027], GO:0004062, GO:0004304, protein-tyrosine sulfotransferase activity [GO:0008476], HNK-1 sulfotransferase activity [GO:0016232], tyrosine-ester sulfotransferase activity [GO:0017067], thiol sulfotransferase activity [GO:0033870], petromyzonol sulfotransferase activity [GO:0033873], scymnol sulfotransferase activity [GO:0033874], glycochenodeoxycholate sulfotransferase activity [GO:0033876], triglucosylalkylacylglycerol sulfotransferase activity [GO:0047363], GO:0047364, GO:0047365, quercetin-3-sulfate 4'-sulfotransferase activity [GO:0047366], GO:0047367, UDP-N-acetylgalactosamine-4-sulfate sulfotransferase activity [GO:0047368], GO:0047685, GO:0047686, bile-salt sulfotransferase activity [GO:0047704], choline sulfotransferase activity [GO:0047754], GO:0047785, flavonol 3-sulfotransferase activity [GO:0047894], psychosine sulfotransferase activity [GO:0050226], Renilla-luciferin sulfotransferase activity [GO:0050249], steroid sulfotransferase activity [GO:0050294], N-acetylgalactosamine 4-sulfate 6-O-sulfotransferase activity [GO:0050659], GO:0050694, GO:0050698, brassinosteroid sulfotransferase activity [GO:0080118], hydroxyjasmonate sulfotransferase activity [GO:0080131], aliphatic desulfoglucosinolate sulfotransferase activity [GO:0120527], flavonoid sulfotransferase activity [GO:1990135] Definition: Catalysis of the transfer of a sulfate group from 3'-phosphoadenosine 5'-phosphosulfate to the hydroxyl group of an acceptor, producing the sulfated derivative and 3'-phosphoadenosine 5'-phosphate.